phosphatidylethanolamine catabolic process [GO:0046338] (biological process) Relationships: is a type of phosphatidylethanolamine metabolic process [GO:0046337]; is a type of GO:0046475 Sources: ISBN:0198506732 Definition: The chemical reactions and pathways resulting in the breakdown of phosphatidylethanolamine, any of a class of glycerophospholipids in which a phosphatidyl group is esterified to the hydroxyl group of ethanolamine. Also known as: phosphatidylethanolamine breakdown, phosphatidylethanolamine catabolism, phosphatidylethanolamine degradation